{
  "term_label": "cytoplasm",
  "gene_name": "Probable ATP-dependent RNA helicase DDX60",
  "gene_symbol": "DDX60",
  "term_id": "GO:0005737",
  "gene": "UniProtKB:Q8IY21"
}